{
  "term_label": "Unknown cellular component",
  "gene_symbol": "IGKJ4",
  "gene": "UniProtKB:A0A0A0MT69",
  "term_id": "UNKNOWN:0003",
  "gene_name": "Immunoglobulin kappa joining 4 (Fragment)"
}